{
  "gene_symbol": "LIMD2",
  "gene_name": "LIM domain-containing protein 2",
  "gene": "UniProtKB:Q9BT23",
  "term_id": "GO:0015629",
  "term_label": "actin cytoskeleton"
}